{
  "term_label": "ATP-dependent diacylglycerol kinase activity",
  "gene_symbol": "DGKH",
  "term_id": "GO:0004143",
  "gene": "UniProtKB:Q86XP1",
  "gene_name": "Diacylglycerol kinase eta"
}